response to lipoprotein particle [GO:0055094] (biological process) Sources: GOC:BHF, GOC:rl Subtypes: cellular response to low-density lipoprotein particle stimulus [GO:0071404], cellular response to very-low-density lipoprotein particle stimulus [GO:0090731] Also known as: response to lipoprotein particle stimulus Definition: Any process that results in a change in state or activity of a cell or an organism (in terms of movement, secretion, enzyme production, gene expression, etc.) as a result of a lipoprotein particle stimulus. Relationships: is a type of response to endogenous stimulus [GO:0009719]; is_a GO:1901698